{
  "term_label": "ATP hydrolysis activity",
  "gene_symbol": "DHX9",
  "gene_name": "ATP-dependent RNA helicase A",
  "gene": "UniProtKB:Q08211",
  "term_id": "GO:0016887"
}